{
  "term_label": "RNA polymerase II cis-regulatory region sequence-specific DNA binding",
  "term_id": "GO:0000978",
  "gene_symbol": "MSGN1",
  "gene_name": "Mesogenin-1",
  "gene": "UniProtKB:A6NI15"
}